{
  "gene_name": "Lysine-specific demethylase RSBN1L",
  "gene": "UniProtKB:Q6PCB5",
  "term_id": "UNKNOWN:0002",
  "gene_symbol": "RSBN1L",
  "term_label": "Unknown biological process"
}